{
  "gene_name": "1-acylglycerol-3-phosphate O-acyltransferase ABHD5",
  "term_id": "GO:0004620",
  "term_label": "phospholipase activity",
  "gene_symbol": "ABHD5",
  "gene": "UniProtKB:Q8WTS1"
}